regulation of epithelial cell-cell adhesion involved in epithelium migration [GO:1903681] (BP) Definition: Any process that modulates the frequency, rate or extent of epithelial cell-cell adhesion involved in epithelium migration. References: PMID:18394891 Sources: GOC:TermGenie, GOC:als, GO_REF:0000058 Relationships: is a type of regulation of cell-cell adhesion [GO:0022407]; is a type of regulation of multicellular organismal process [GO:0051239]; regulates GO:0090137 Subtypes: negative regulation of epithelial cell-cell adhesion involved in epithelium migration [GO:1903682], GO:1903683